{
  "gene_name": "Actin-related protein 2_3 complex subunit 3",
  "term_label": "actin filament binding",
  "gene_symbol": "ARPC3",
  "term_id": "GO:0051015",
  "gene": "UniProtKB:O15145"
}